(+)-pulegone reductase (NADP+) activity [GO:0052579] (molecular function) Relationships: is a type of oxidoreductase activity, acting on the CH-CH group of donors, NAD or NADP as acceptor [GO:0016628] Sources: EC:1.3.1.81 Definition: Catalysis of the reaction: (1R,4S)-menthone + NADP+ = (R)-pulegone + H+ + NADPH. Also converts (2R,5R)-isomenthone into (R)-pulegone. Also known as: (+)-isomenthone:NADP+ oxidoreductase activity